{
  "gene_symbol": "NCR3LG1",
  "term_label": "Unknown biological process",
  "gene_name": "Natural cytotoxicity triggering receptor 3 ligand 1",
  "gene": "UniProtKB:Q68D85",
  "term_id": "UNKNOWN:0002"
}